cGMP binding [GO:0030553] (molecular function) Sources: GOC:ai Definition: Binding to cGMP, the nucleotide cyclic GMP (guanosine 3',5'-cyclophosphate). Also known as: 3',5' cGMP binding, 3',5'-cGMP binding, cyclic GMP binding Relationships: is a type of cyclic nucleotide binding [GO:0030551]; is a type of guanyl ribonucleotide binding [GO:0032561]; is a type of GO:0043168